oxidoreductase activity, acting on the CH-NH2 group of donors, with a copper protein as acceptor [GO:0052877] (molecular function) Definition: Catalysis of an oxidation-reduction (redox) reaction in which a CH-NH2 group acts as a hydrogen or electron donor and a copper protein is the acceptor. Sources: GOC:ai Relationships: is a type of oxidoreductase activity, acting on the CH-NH2 group of donors [GO:0016638] Subtypes: aralkylamine dehydrogenase (azurin) activity [GO:0030059], methylamine dehydrogenase (amicyanin) activity [GO:0052876]